{
  "gene": "UniProtKB:A0A0G2JMM0",
  "term_label": "transmembrane signaling receptor activity",
  "gene_symbol": "LOC128966728",
  "gene_name": "Uncharacterized protein",
  "term_id": "GO:0004888"
}